{
  "gene_symbol": "ASIC4",
  "term_label": "ligand-gated sodium channel activity",
  "gene": "UniProtKB:Q96FT7",
  "gene_name": "Acid-sensing ion channel 4",
  "term_id": "GO:0015280"
}